{
  "term_id": "UNKNOWN:0001",
  "term_label": "Unknown molecular function",
  "gene_symbol": "IGHD5OR15-5B",
  "gene_name": "Immunoglobulin heavy diversity 5_OR15-5A (non-functional) (Fragment)",
  "gene": "UniProtKB:A0A0G2JLJ8"
}